regulation of transcription from RNA polymerase II promoter by galactose [GO:0000431] (biological process) Definition: Any process involving galactose that modulates the frequency, rate or extent of transcription from an RNA polymerase II promoter. Subtypes: GO:0000434, positive regulation of transcription from RNA polymerase II promoter by galactose [GO:0000435] Sources: GOC:krc Relationships: is a type of regulation of transcription by galactose [GO:0000409]; is a type of GO:0000429